positive regulation of flower development [GO:0009911] (biological process) Definition: Any process that activates or increases the frequency, rate or extent of flower development. Sources: GOC:go_curators Also known as: up regulation of flower development, up-regulation of flower development, upregulation of flower development, activation of flower development, stimulation of flower development Relationships: is_a regulation of flower development [GO:0009909]; is a type of positive regulation of post-embryonic development [GO:0048582]; is a type of positive regulation of reproductive process [GO:2000243]; positively regulates flower development [GO:0009908]